{
  "term_id": "GO:0005829",
  "gene_name": "Protein FAM83D",
  "term_label": "cytosol",
  "gene": "UniProtKB:Q9H4H8",
  "gene_symbol": "FAM83D"
}